{
  "term_id": "GO:0005634",
  "gene_symbol": "ZSCAN10",
  "gene": "UniProtKB:Q96SZ4",
  "gene_name": "Zinc finger and SCAN domain-containing protein 10",
  "term_label": "nucleus"
}